{
  "gene_symbol": "IGHE",
  "gene": "UniProtKB:P01854",
  "term_id": "GO:0006958",
  "gene_name": "Immunoglobulin heavy constant epsilon",
  "term_label": "complement activation, classical pathway"
}